{
  "term_label": "Unknown molecular function",
  "gene_name": "Proline-rich protein 12",
  "gene_symbol": "PRR12",
  "gene": "UniProtKB:Q9ULL5",
  "term_id": "UNKNOWN:0001"
}